{
  "term_label": "endoplasmic reticulum membrane",
  "term_id": "GO:0005789",
  "gene": "UniProtKB:Q6NUK4",
  "gene_name": "Receptor expression-enhancing protein 3",
  "gene_symbol": "REEP3"
}